{
  "gene_symbol": "OR51B5",
  "term_label": "plasma membrane",
  "gene": "UniProtKB:Q9H339",
  "term_id": "GO:0005886",
  "gene_name": "Olfactory receptor 51B5"
}